{
  "gene": "UniProtKB:Q9P1W9",
  "gene_name": "Serine_threonine-protein kinase pim-2",
  "term_label": "cytoplasm",
  "gene_symbol": "PIM2",
  "term_id": "GO:0005737"
}